positive regulation of dephosphorylation [GO:0035306] (biological process) Also known as: up regulation of dephosphorylation, up-regulation of dephosphorylation, upregulation of dephosphorylation, activation of dephosphorylation, stimulation of dephosphorylation Relationships: is a type of regulation of dephosphorylation [GO:0035303]; is a type of GO:0045937; positively regulates GO:0016311 Subtypes: positive regulation of phosphatase activity [GO:0010922] Definition: Any process that activates or increases the frequency, rate or extent of removal of phosphate groups from a molecule. Sources: GOC:bf